{
  "gene_symbol": "MPP3",
  "term_id": "GO:0005911",
  "term_label": "cell-cell junction",
  "gene_name": "MAGUK p55 subfamily member 3",
  "gene": "UniProtKB:Q13368"
}